nucleic acid conformation isomerase activity [GO:0120545] (molecular function) Relationships: is a type of macromolecular conformation isomerase activity [GO:0120543] Sources: EC:5.6.2.- Subtypes: DNA topoisomerase activity [GO:0003916], helicase activity [GO:0004386], RNA topoisomerase activity [GO:0140226], annealing activity [GO:0140666] Definition: Catalysis of a reaction that alters the conformation of a nucleic acid.